{
  "gene": "UniProtKB:Q9BYE3",
  "term_label": "Unknown biological process",
  "gene_name": "Late cornified envelope protein 3D",
  "gene_symbol": "LCE3D",
  "term_id": "UNKNOWN:0002"
}